{
  "gene_symbol": "HCN1",
  "term_label": "sodium ion transmembrane transport",
  "gene": "UniProtKB:O60741",
  "gene_name": "Potassium_sodium hyperpolarization-activated cyclic nucleotide-gated channel 1",
  "term_id": "GO:0035725"
}